{
  "gene_symbol": "LMO3",
  "term_id": "GO:0045944",
  "term_label": "positive regulation of transcription by RNA polymerase II",
  "gene_name": "LIM domain only protein 3",
  "gene": "UniProtKB:Q8TAP4"
}